four-way junction DNA binding [GO:0000400] (molecular function) Relationships: is a type of DNA secondary structure binding [GO:0000217] Definition: Binding to a DNA segment containing four-way junctions, also known as Holliday junctions, a structure where two DNA double strands are held together by reciprocal exchange of two of the four strands, one strand each from the two original helices. Also known as: forked DNA binding, Holliday junction binding References: PMID:15563464 Sources: GOC:krc, ISBN:0815332181 Subtypes: GO:0000401, crossed form four-way junction DNA binding [GO:0000402]